neuronal action potential [GO:0019228] (biological process) Sources: GOC:dph, GOC:isa_complete, GOC:tb Relationships: is a type of action potential [GO:0001508]; is part of transmission of nerve impulse [GO:0019226] Also known as: generation of action potential Regulation: regulated by regulation of neuronal action potential [GO:0098908]; negatively regulated by negative regulation of neuronal action potential [GO:1904456]; positively regulated by positive regulation of neuronal action potential [GO:1904457] Definition: An action potential that occurs in a neuron.